{
  "gene_name": "Transcription factor AP-4",
  "term_id": "GO:0000978",
  "gene": "UniProtKB:Q01664",
  "gene_symbol": "TFAP4",
  "term_label": "RNA polymerase II cis-regulatory region sequence-specific DNA binding"
}